{
  "gene": "UniProtKB:Q14324",
  "term_label": "structural constituent of muscle",
  "gene_symbol": "MYBPC2",
  "term_id": "GO:0008307",
  "gene_name": "Myosin-binding protein C, fast-type"
}